{
  "gene": "UniProtKB:Q9Y4B4",
  "term_label": "ATP-dependent chromatin remodeler activity",
  "gene_name": "Helicase ARIP4",
  "term_id": "GO:0140658",
  "gene_symbol": "RAD54L2"
}